{
  "term_id": "GO:0006749",
  "gene_symbol": "GSR",
  "term_label": "glutathione metabolic process",
  "gene_name": "Glutathione reductase, mitochondrial",
  "gene": "UniProtKB:P00390"
}